{
  "gene_symbol": "FSD1",
  "term_id": "GO:0051302",
  "gene_name": "Fibronectin type III and SPRY domain-containing protein 1",
  "term_label": "regulation of cell division",
  "gene": "UniProtKB:Q9BTV5"
}